pseudouridine kinase activity [GO:0050225] (molecular function) Definition: Catalysis of the reaction: ATP + pseudouridine = ADP + 2 H+ + pseudouridine 5'-phosphate. Sources: EC:2.7.1.83, RHEA:22448 Also known as: ATP:pseudouridine 5'-phosphotransferase activity, pseudouridine kinase (phosphorylating) Relationships: is a type of kinase activity [GO:0016301]; is a type of phosphotransferase activity, alcohol group as acceptor [GO:0016773]